{
  "term_id": "UNKNOWN:0001",
  "gene_symbol": "HMMR",
  "term_label": "Unknown molecular function",
  "gene_name": "Hyaluronan mediated motility receptor",
  "gene": "UniProtKB:O75330"
}